{
  "term_id": "GO:0005737",
  "gene_name": "Volume-regulated anion channel subunit LRRC8D",
  "gene_symbol": "LRRC8D",
  "term_label": "cytoplasm",
  "gene": "UniProtKB:Q7L1W4"
}